{
  "gene_symbol": "ZNF566",
  "gene_name": "Zinc finger protein 566",
  "term_label": "nucleus",
  "gene": "UniProtKB:Q969W8",
  "term_id": "GO:0005634"
}